{
  "gene_name": "CD177 antigen",
  "term_id": "GO:0045217",
  "term_label": "cell-cell junction maintenance",
  "gene_symbol": "CD177",
  "gene": "UniProtKB:Q8N6Q3"
}